{
  "term_label": "extracellular space",
  "term_id": "GO:0005615",
  "gene_symbol": "FCN2",
  "gene_name": "Ficolin-2",
  "gene": "UniProtKB:Q15485"
}